{
  "gene_name": "Acetylcholine receptor subunit beta",
  "term_label": "synaptic transmission, cholinergic",
  "gene_symbol": "CHRNB1",
  "term_id": "GO:0007271",
  "gene": "UniProtKB:P11230"
}